RNA polymerase II C-terminal domain O-GlcNAc transferase activity [GO:0140841] (molecular function) References: PMID:22605332 Relationships: is a type of protein O-acetylglucosaminyltransferase activity [GO:0097363] Subtypes: RNA polymerase II C-terminal domain S5 O-GlcNAc transferase activity [GO:0140842], RNA polymerase II C-terminal domain S7 O-GlcNAc transferase activity [GO:0140843] Definition: Catalysis of the reaction: UDP-N-acetyl-D-glucosamine + RNA polymerase II large subunit CTD heptapeptide repeat (YSPTSPS) = UDP + RNA polymerase II large subunit CTD heptapeptide repeat 3-O-(N-acetyl-D-glucosaminyl)-L-serine.